{
  "term_id": "GO:0003682",
  "gene_name": "Bromodomain-containing protein 4",
  "gene": "UniProtKB:O60885",
  "term_label": "chromatin binding",
  "gene_symbol": "BRD4"
}